3'-phospho-5'-adenylyl sulfate transmembrane transport [GO:1902559] (biological process) Relationships: is a type of 3'-phosphoadenosine 5'-phosphosulfate transport [GO:0046963]; is a type of purine-containing compound transmembrane transport [GO:0072530]; is a type of GO:1901679 References: PMID:24296033 Sources: GOC:TermGenie Subtypes: mitochondrial 3'-phospho-5'-adenylyl sulfate transmembrane transport [GO:1990554] Also known as: 3'-phosphoadenosine 5'-phosphosulfate transmembrane transport Definition: The process in which 3'-phospho-5'-adenylyl sulfate is transported across a membrane.